cellular response to bacteriocin [GO:0071237] (biological process) Definition: Any process that results in a change in state or activity of a cell (in terms of movement, secretion, enzyme production, gene expression, etc.) as a result of a bacteriocin stimulus. A bacteriocin is a protein substance released by certain bacteria that kills but does not lyse closely related strains of bacteria. Specific bacteriocins attach to specific receptors on cell walls and induce specific metabolic block, e.g. cessation of nucleic acid or protein synthesis of oxidative phosphorylation. Sources: GOC:mah Relationships: is a type of GO:0046678; is a type of cellular response to antibiotic [GO:0071236]; is a type of cellular response to nitrogen compound [GO:1901699]; is a type of cellular response to oxygen-containing compound [GO:1901701]